{
  "gene_name": "ATP-dependent RNA helicase DHX15",
  "term_id": "GO:0003723",
  "gene_symbol": "DHX15",
  "term_label": "RNA binding",
  "gene": "UniProtKB:O43143"
}